trans-zeatin biosynthetic process [GO:0033466] (biological process) Sources: GOC:mah Relationships: is a type of zeatin biosynthetic process [GO:0033398] Also known as: trans-zeatin anabolism, trans-zeatin biosynthesis, trans-zeatin formation, trans-zeatin synthesis Definition: The chemical reactions and pathways resulting in the formation of trans-zeatin, (2E)-2-methyl-4-(9H-purin-6-ylamino)but-2-en-1-ol.